mitochondrial ribosome assembly [GO:0061668] (biological process) Sources: GOC:dph Relationships: is a type of ribosome assembly [GO:0042255] Definition: The aggregation, arrangement and bonding together of the mitochondrial ribosome and of its subunits.